{
  "term_label": "Unknown molecular function",
  "gene": "UniProtKB:Q969Q6",
  "gene_symbol": "PPP2R3C",
  "gene_name": "Serine_threonine-protein phosphatase 2A regulatory subunit B'' subunit gamma",
  "term_id": "UNKNOWN:0001"
}